immature T cell proliferation in thymus [GO:0033080] (biological process) Relationships: is a type of immature T cell proliferation [GO:0033079]; is part of T cell differentiation in thymus [GO:0033077] Regulation: regulated by regulation of immature T cell proliferation in thymus [GO:0033084]; negatively regulated by GO:0033088; positively regulated by positive regulation of immature T cell proliferation in thymus [GO:0033092] Also known as: thymic T cell proliferation, thymocyte cell proliferation, thymocyte proliferation Sources: GOC:add, ISBN:0781735149 Definition: The expansion of an immature T cell population by cell division in the thymus.